{
  "gene": "UniProtKB:O60548",
  "gene_symbol": "FOXD2",
  "term_label": "cell differentiation",
  "gene_name": "Forkhead box protein D2",
  "term_id": "GO:0030154"
}